{
  "term_label": "L-glutamine catabolic process",
  "gene": "UniProtKB:O94925",
  "gene_symbol": "GLS",
  "term_id": "GO:0006543",
  "gene_name": "Glutaminase kidney isoform, mitochondrial"
}